{
  "term_id": "GO:0030425",
  "gene": "UniProtKB:P47898",
  "term_label": "dendrite",
  "gene_symbol": "HTR5A",
  "gene_name": "5-hydroxytryptamine receptor 5A"
}